{
  "gene_name": "Nucleotide-binding oligomerization domain-containing protein 2",
  "term_label": "pattern recognition receptor activity",
  "gene_symbol": "NOD2",
  "term_id": "GO:0038187",
  "gene": "UniProtKB:Q9HC29"
}